{
  "term_label": "methionine biosynthetic process",
  "term_id": "GO:0009086",
  "gene_symbol": "MTHFR",
  "gene_name": "Methylenetetrahydrofolate reductase (NADPH)",
  "gene": "UniProtKB:P42898"
}